{
  "gene_name": "Metallothionein-1L",
  "gene_symbol": "MT1L",
  "term_id": "GO:0071280",
  "term_label": "cellular response to copper ion",
  "gene": "UniProtKB:Q93083"
}